{
  "gene": "UniProtKB:Q6ZNA1",
  "gene_name": "Zinc finger protein 836",
  "term_id": "GO:0000976",
  "term_label": "transcription cis-regulatory region binding",
  "gene_symbol": "ZNF836"
}